{
  "term_label": "Unknown cellular component",
  "term_id": "UNKNOWN:0003",
  "gene_symbol": "CLSPN",
  "gene": "UniProtKB:Q9HAW4",
  "gene_name": "Claspin"
}